clathrin-sculpted monoamine transport vesicle lumen [GO:0070082] (CC) Also known as: clathrin sculpted monoamine constitutive secretory pathway transport vesicle lumen, clathrin sculpted monoamine transport vesicle lumen Relationships: is a type of cytoplasmic vesicle lumen [GO:0060205]; BFO_0000050 clathrin-sculpted monoamine transport vesicle [GO:0070081] Sources: GOC:mg2 Definition: The volume enclosed by the membrane of the clathrin-sculpted monoamine transport vesicle.